epithelium migration involved in imaginal disc-derived wing morphogenesis [GO:0090252] (biological process) Definition: The process in which the population of cells that make up a wing epithelium undergo directed movement and contribute to imaginal disc-derived morphogenesis. Sources: GOC:ascb_2009, GOC:dph, GOC:tb Relationships: is a type of epithelium migration [GO:0090132]; is part of imaginal disc-derived wing morphogenesis [GO:0007476]